{
  "term_label": "axonogenesis",
  "gene": "UniProtKB:P63261",
  "gene_symbol": "ACTG1",
  "term_id": "GO:0007409",
  "gene_name": "Actin, cytoplasmic 2"
}